Hrd1p ubiquitin ligase complex [GO:0000836] (cellular component) Also known as: HRD1 ubiquitin ligase complex References: PMID:16619026, PMID:16873066, PMID:21454652 Sources: GOC:bf, GOC:elh Subtypes: GO:0000838, Hrd1p ubiquitin ligase ERAD-L complex [GO:0000839] Definition: A multiprotein complex that recognizes and ubiquitinates proteins with misfolded luminal and membrane domains during ER-associated protein degradation (ERAD). In S. cerevisiae, this complex contains the ubiquitin ligase Hrd1p. In mammals, this complex contains the ubiquitin ligase HRD1 (Synoviolin) or AMFR (gp78). Relationships: is a type of GO:0000835